{
  "gene_name": "Histone H2B type 1-O",
  "gene": "UniProtKB:P23527",
  "term_id": "GO:0000786",
  "term_label": "nucleosome",
  "gene_symbol": "H2BC17"
}